L-kynurenine catabolic process [GO:0097053] (biological process) Relationships: is a type of ketone catabolic process [GO:0042182]; is a type of L-kynurenine metabolic process [GO:0097052]; is a type of L-amino acid catabolic process [GO:0170035]; is a type of non-proteinogenic amino acid catabolic process [GO:0170044] Sources: GOC:yaf Also known as: L-kynurenine breakdown, L-kynurenine catabolism, L-kynurenine degradation Definition: The chemical reactions and pathways resulting in the breakdown of L-kynurenine, the L-enantiomer of the amino acid kynurenine (3-(2-aminobenzoyl)-alanine).